{
  "gene": "UniProtKB:O60779",
  "term_id": "GO:0015234",
  "term_label": "thiamine transmembrane transporter activity",
  "gene_name": "Thiamine transporter 1",
  "gene_symbol": "SLC19A2"
}